{
  "term_label": "nervous system development",
  "gene": "UniProtKB:Q7Z6B7",
  "term_id": "GO:0007399",
  "gene_symbol": "SRGAP1",
  "gene_name": "SLIT-ROBO Rho GTPase-activating protein 1"
}